pyrimidine-containing compound salvage [GO:0008655] (biological process) Sources: GOC:jl Also known as: pyrimidine salvage Subtypes: GO:0032262, GO:0036172, pyrimidine nucleoside salvage [GO:0043097], pyrimidine nucleobase salvage [GO:0043100] Regulation: regulated by regulation of pyrimidine-containing compound salvage [GO:1903930]; positively regulated by GO:1903931 Relationships: is a type of metabolic compound salvage [GO:0043094]; is a type of pyrimidine-containing compound biosynthetic process [GO:0072528] Definition: Any process that generates a pyrimidine-containing compound, a nucleobase, nucleoside, nucleotide or nucleic acid that contains a pyrimidine base, from derivatives of them without de novo synthesis.